{
  "gene": "UniProtKB:Q86YV9",
  "term_id": "UNKNOWN:0001",
  "gene_name": "BLOC-2 complex member HPS6",
  "gene_symbol": "HPS6",
  "term_label": "Unknown molecular function"
}